{
  "gene_symbol": "KRT28",
  "term_label": "epithelial cell differentiation",
  "gene": "UniProtKB:Q7Z3Y7",
  "term_id": "GO:0030855",
  "gene_name": "Keratin, type I cytoskeletal 28"
}